circadian regulation of gene expression [GO:0032922] (biological process) Relationships: is a type of circadian rhythm [GO:0007623]; is a type of regulation of gene expression [GO:0010468] Sources: GOC:mah Also known as: circadian regulation of protein expression, diurnal variation of gene expression, diurnal variation of protein expression Definition: Any process that modulates the frequency, rate or extent of gene expression such that an expression pattern recurs with a regularity of approximately 24 hours.